{
  "gene": "UniProtKB:O76083",
  "term_label": "3',5'-cyclic-GMP phosphodiesterase activity",
  "term_id": "GO:0047555",
  "gene_symbol": "PDE9A",
  "gene_name": "High affinity cGMP-specific 3',5'-cyclic phosphodiesterase 9A"
}